{
  "gene_name": "Eukaryotic translation initiation factor 2A",
  "gene": "UniProtKB:Q9BY44",
  "gene_symbol": "EIF2A",
  "term_id": "GO:0003743",
  "term_label": "translation initiation factor activity"
}